D-lactate dehydrogenase (cytochrome) activity [GO:0004458] (molecular function) Definition: Catalysis of the reaction: (R)-lactate + 2 [Fe(III)cytochrome c] = 2 [Fe(II)cytochrome c] + 2 H+ + pyruvate. Sources: RHEA:13521 Relationships: is a type of oxidoreductase activity, acting on the CH-OH group of donors, cytochrome as acceptor [GO:0016898]; is a type of D-lactate dehydrogenase activity [GO:0047809] Also known as: D-lactate dehydrogenase activity, lactic acid dehydrogenase activity, (R)-lactate:ferricytochrome-c 2-oxidoreductase activity, D-(-)-lactic cytochrome c reductase activity, D-lactate (cytochrome) dehydrogenase activity, D-lactate ferricytochrome c oxidoreductase activity, D-lactate-cytochrome c reductase activity, cytochrome-dependent D-(-)-lactate dehydrogenase activity